{
  "term_id": "GO:0043588",
  "gene_name": "Collagen alpha-2(V) chain",
  "term_label": "skin development",
  "gene_symbol": "COL5A2",
  "gene": "UniProtKB:P05997"
}